{
  "gene": "UniProtKB:Q9NQX6",
  "term_id": "GO:0006355",
  "gene_symbol": "ZNF331",
  "gene_name": "Zinc finger protein 331",
  "term_label": "regulation of DNA-templated transcription"
}